UDP-glucose 4-epimerase activity [GO:0003978] (molecular function) Definition: Catalysis of the reaction: UDP-glucose = UDP-galactose. Also known as: 4-epimerase activity, UDP-D-galactose 4-epimerase activity, UDP-galactose 4-epimerase activity, UDP-glucose epimerase activity, UDPG-4-epimerase activity, UDPgalactose 4-epimerase activity, UDPglucose 4-epimerase activity, galactowaldenase activity, uridine diphosphate galactose 4-epimerase activity, uridine diphosphate glucose 4-epimerase activity, uridine diphospho-galactose-4-epimerase activity, uridine diphosphoglucose 4-epimerase activity, uridine diphosphoglucose epimerase activity Sources: EC:5.1.3.2 Relationships: is a type of racemase and epimerase activity, acting on carbohydrates and derivatives [GO:0016857]